cortical microtubule [GO:0055028] (cellular component) Relationships: is a type of cytoplasmic microtubule [GO:0005881]; is part of GO:0030981 Definition: Arrays of microtubules underlying and connected to the plasma membrane in the cortical cytosol. Subtypes: cortical microtubule, transverse to long axis [GO:0010005] Sources: GOC:mtg_sensu